{
  "gene": "UniProtKB:P33151",
  "gene_symbol": "CDH5",
  "term_label": "adherens junction",
  "gene_name": "Cadherin-5",
  "term_id": "GO:0005912"
}